{
  "gene_name": "Testis-specific protein LINC02914",
  "gene_symbol": "LINC02914",
  "term_id": "UNKNOWN:0001",
  "gene": "UniProtKB:Q52M58",
  "term_label": "Unknown molecular function"
}